{
  "gene": "UniProtKB:P55291",
  "term_label": "cell-cell adhesion mediated by cadherin",
  "gene_symbol": "CDH15",
  "term_id": "GO:0044331",
  "gene_name": "Cadherin-15"
}